{
  "term_label": "voltage-gated potassium channel complex",
  "term_id": "GO:0008076",
  "gene_name": "Leucine-rich repeat-containing protein 38",
  "gene": "UniProtKB:Q5VT99",
  "gene_symbol": "LRRC38"
}